{
  "gene": "UniProtKB:P21854",
  "term_id": "UNKNOWN:0002",
  "gene_symbol": "CD72",
  "term_label": "Unknown biological process",
  "gene_name": "B-cell differentiation antigen CD72"
}